MsbA transporter complex [GO:1990199] (cellular component) Also known as: MsbA complex, MsbA dimer Definition: An ATP-binding cassette (ABC) transporter complex made up of a dimer of MsbA. Facilitates the export across the plasma membrane of, amongst others, lipid A and lipopolysaccharide. In contrast to most ABC transporter complexes, each chain of the homodimer contains both the transmembrane domain (TMD) and the cytoplasmic ATP-binding domain (NBD). References: PMID:18024585 Sources: GOC:bhm Relationships: is a type of ATP-binding cassette (ABC) transporter complex [GO:0043190]